{
  "term_label": "Unknown cellular component",
  "gene": "UniProtKB:O95848",
  "gene_name": "Uridine diphosphate glucose pyrophosphatase NUDT14",
  "term_id": "UNKNOWN:0003",
  "gene_symbol": "NUDT14"
}